laminin-14 complex [GO:1990338] (cellular component) References: PMID:15979864, PMID:17453709 Sources: GOC:bhm, GOC:dph Also known as: laminin-423 Relationships: is a type of laminin complex [GO:0043256] Definition: A laminin complex composed of alpha4, beta2 and gamma3 polypeptide chains.